{
  "gene": "UniProtKB:Q86YL7",
  "term_id": "GO:0007165",
  "term_label": "signal transduction",
  "gene_symbol": "PDPN",
  "gene_name": "Podoplanin"
}